aminoacyl-tRNA metabolism involved in translational fidelity [GO:0106074] (biological process) Relationships: is a type of tRNA metabolic process [GO:0006399]; is a type of GO:0006450 Sources: GOC:hjd Also known as: aminoacyl-tRNA correction, aminoacyl-tRNA editin, aminoacyl-tRNA proofreading Definition: Any process which detects an amino-acid acetylated tRNA is charged with the correct amino acid, or removes incorrect amino acids from a charged tRNA. This process can be performed by tRNA synthases, or by subsequent reactions after tRNA aminoacylation.